microtubule-based transport [GO:0099111] (biological process) Relationships: is a type of transport [GO:0006810] Definition: A microtubule-based process that results in the transport of organelles, other microtubules, or other cellular components. Examples include motor-driven movement along microtubules and movement driven by polymerization or depolymerization of microtubules. Subtypes: epithelial cilium movement involved in extracellular fluid movement [GO:0003351], transport along microtubule [GO:0010970], nuclear migration by microtubule mediated pushing forces [GO:0098863], microtubule-based protein transport [GO:0099118] Sources: GOC:cjm, ISBN:0815316194